{
  "gene_symbol": "CYP1A1",
  "gene": "UniProtKB:P04798",
  "term_id": "GO:0016712",
  "term_label": "oxidoreductase activity, acting on paired donors, with incorporation or reduction of molecular oxygen, reduced flavin or flavoprotein as one donor, and incorporation of one atom of oxygen",
  "gene_name": "Cytochrome P450 1A1"
}